{
  "gene_name": "Immunoglobulin kappa variable 5-2",
  "term_id": "UNKNOWN:0001",
  "gene": "UniProtKB:P06315",
  "gene_symbol": "IGKV5-2",
  "term_label": "Unknown molecular function"
}